{
  "gene_name": "Axin-1",
  "term_label": "I-SMAD binding",
  "gene_symbol": "AXIN1",
  "term_id": "GO:0070411",
  "gene": "UniProtKB:O15169"
}